{
  "gene": "UniProtKB:Q92506",
  "term_label": "fatty acid biosynthetic process",
  "gene_symbol": "HSD17B8",
  "term_id": "GO:0006633",
  "gene_name": "(3R)-3-hydroxyacyl-CoA dehydrogenase"
}